regulation of type IIb hypersensitivity [GO:0001799] (biological process) Definition: Any process that modulates the frequency, rate, or extent of type IIb hypersensitivity, a type of inflammatory response. Relationships: is a type of regulation of type II hypersensitivity [GO:0002892]; regulates type IIb hypersensitivity [GO:0001795] Subtypes: negative regulation of type IIb hypersensitivity [GO:0001800], positive regulation of type IIb hypersensitivity [GO:0001801] Sources: GOC:add, ISBN:0781735149